{
  "term_id": "GO:0051726",
  "gene": "UniProtKB:Q13490",
  "gene_symbol": "BIRC2",
  "gene_name": "Baculoviral IAP repeat-containing protein 2",
  "term_label": "regulation of cell cycle"
}